{
  "gene_name": "POU domain, class 6, transcription factor 1",
  "term_label": "regulation of transcription by RNA polymerase II",
  "term_id": "GO:0006357",
  "gene_symbol": "POU6F1",
  "gene": "UniProtKB:Q14863"
}